Kir2 inward rectifier potassium channel complex [GO:1990374] (cellular component) Also known as: Kir2.1 complex Definition: A inward rectifier potassium channel complex. Homo- or heterotetramer composed of subunits of the eukaryotic Kir2 protein family. Plays a key role in maintaining the correct resting potential in eukaryotic cells. References: PMID:16834334 Sources: GOC:bhm Note: An example of this is Kcnj2 in mouse (P35561) in PMID:16834334 (inferred from direct assay). Relationships: is_a inward rectifier potassium channel complex [GO:1902937]